AMPA glutamate receptor clustering [GO:0097113] (biological process) Regulation: regulated by regulation of AMPA glutamate receptor clustering [GO:1904717]; negatively regulated by GO:1904718; positively regulated by positive regulation of AMPA glutamate receptor clustering [GO:1904719] Definition: The glutamate receptor clustering process in which alpha-amino-3-hydroxy-5-methyl-4-isoxazole propionate (AMPA) receptors are localized to distinct domains in the cell membrane. Also known as: AMPA receptor clustering, alpha-amino-3-hydroxy-5-methyl-4-isoxazole propionate selective glutamate receptor clustering Relationships: is a type of glutamate receptor clustering [GO:0097688]; is part of GO:0001941 References: PMID:12796785 Sources: GOC:BHF, GOC:pr, GOC:sjp